cell cortex [GO:0005938] (cellular component) Also known as: ectoplasm, cell periphery, peripheral cytoplasm Subtypes: cell cortex region [GO:0099738] Definition: The region of a cell that lies just beneath the plasma membrane and often, but not always, contains a network of actin filaments and associated proteins. Relationships: is a type of cytoplasm [GO:0005737]; is part of cell periphery [GO:0071944] Sources: GOC:mah, ISBN:0815316194